{
  "term_id": "GO:0030490",
  "gene": "UniProtKB:O14730",
  "term_label": "maturation of SSU-rRNA",
  "gene_name": "Serine_threonine-protein kinase RIO3",
  "gene_symbol": "RIOK3"
}